{
  "gene": "UniProtKB:Q6PEY2",
  "gene_symbol": "TUBA3E",
  "gene_name": "Tubulin alpha-3E chain",
  "term_label": "cytoplasm",
  "term_id": "GO:0005737"
}